{
  "gene_name": "Keratin-associated protein 6-1",
  "term_label": "Unknown molecular function",
  "term_id": "UNKNOWN:0001",
  "gene": "UniProtKB:Q3LI64",
  "gene_symbol": "KRTAP6-1"
}